{
  "gene_name": "Striatin",
  "term_label": "protein-macromolecule adaptor activity",
  "gene_symbol": "STRN",
  "gene": "UniProtKB:O43815",
  "term_id": "GO:0030674"
}